1-phosphatidylinositol-3-kinase activity [GO:0016303] (molecular function) Relationships: is a type of GO:0052742; BFO_0000050 phosphatidylinositol-3-phosphate biosynthetic process [GO:0036092] Definition: Catalysis of the reaction: a 1-phosphatidyl-1D-myo-inositol + ATP = a 1-phosphatidyl-1D-myo-inositol 3-phosphate + ADP + H+. Also known as: 1-phosphatidylinositol 3-kinase activity, PI3-kinase activity, PI3K, PtdIns-3-kinase activity, phosphatidylinositol 3-kinase activity, class I, phosphatidylinositol 3-kinase activity, class II, phosphatidylinositol 3-kinase activity, class III, phosphatidylinositol 3-kinase, class I, catalyst activity, type I phosphatidylinositol kinase activity, type III phosphoinositide 3-kinase activity Sources: EC:2.7.1.137, RHEA:12709 Regulation: regulated by GO:0046935